regulation of type IV pilus biogenesis [GO:1903656] (biological process) Also known as: regulation of TFP biogenesis, regulation of type 4 pilus biogenesis, regulation of type IV fimbria assembly, regulation of type IV fimbria biogenesis, regulation of type IV fimbriae assembly, regulation of type IV fimbriae biogenesis, regulation of type IV fimbrial assembly, regulation of type IV fimbrial biogenesis, regulation of type IV fimbrium assembly, regulation of type IV fimbrium biogenesis, regulation of type IV pilus biosynthesis Subtypes: negative regulation of type IV pilus biogenesis [GO:1903657], positive regulation of type IV pilus biogenesis [GO:1903658] Definition: Any process that modulates the frequency, rate or extent of type IV pilus biogenesis. References: PMID:25049409 Sources: GOC:TermGenie, GO_REF:0000058 Relationships: is a type of regulation of cell projection assembly [GO:0060491]; regulates type IV pilus assembly [GO:0043683]